{
  "gene_name": "BTB_POZ domain-containing protein 3",
  "term_id": "GO:0022008",
  "gene_symbol": "BTBD3",
  "term_label": "neurogenesis",
  "gene": "UniProtKB:Q9Y2F9"
}